positive regulation of microvillus assembly [GO:1903698] (biological process) Definition: Any process that activates or increases the frequency, rate or extent of microvillus assembly. References: PMID:22797597 Sources: GOC:TermGenie, GOC:als, GO_REF:0000058 Relationships: is a type of GO:0032534; is a type of positive regulation of plasma membrane bounded cell projection assembly [GO:0120034]; positively regulates microvillus assembly [GO:0030033] Also known as: up regulation of microvillus assembly, up-regulation of microvillus assembly, upregulation of microvillus assembly, activation of microvillus assembly, activation of microvillus biogenesis, positive regulation of microvillus biogenesis, up regulation of microvillus biogenesis, up-regulation of microvillus biogenesis, upregulation of microvillus biogenesis